peptidoglycan metabolic process [GO:0000270] (biological process) Also known as: murein metabolic process, murein metabolism, peptidoglycan metabolism References: PMID:33139480 Subtypes: GO:0009252, peptidoglycan catabolic process [GO:0009253], GO:0009254 Relationships: is a type of GO:0030203 Definition: The chemical reactions and pathways involving peptidoglycans, any of a class of glycoconjugates found only in bacterial cell walls and consisting of long glycan strands of alternating residues of beta-(1,4) linked N-acetylglucosamine and N-acetylmuramic acid, cross-linked by short peptides.